{
  "term_label": "Unknown biological process",
  "gene_symbol": "DCSTAMP",
  "term_id": "UNKNOWN:0002",
  "gene_name": "Dendritic cell-specific transmembrane protein",
  "gene": "UniProtKB:Q9H295"
}